{
  "gene_name": "HERV-H_2q24.3 provirus ancestral Env polyprotein",
  "gene_symbol": "Q9N2K0",
  "term_label": "Unknown biological process",
  "gene": "UniProtKB:Q9N2K0",
  "term_id": "UNKNOWN:0002"
}